{
  "gene": "UniProtKB:Q96MS0",
  "term_label": "axon guidance",
  "gene_name": "Roundabout homolog 3",
  "term_id": "GO:0007411",
  "gene_symbol": "ROBO3"
}